{
  "term_label": "Unknown biological process",
  "term_id": "UNKNOWN:0002",
  "gene_symbol": "PPM1J",
  "gene_name": "Protein phosphatase 1J",
  "gene": "UniProtKB:Q5JR12"
}